{
  "term_id": "GO:0045910",
  "term_label": "negative regulation of DNA recombination",
  "gene_name": "Regulator of telomere elongation helicase 1",
  "gene": "UniProtKB:Q9NZ71",
  "gene_symbol": "RTEL1"
}